{
  "gene": "UniProtKB:Q9NQ33",
  "gene_name": "Achaete-scute homolog 3",
  "term_label": "positive regulation of transcription by RNA polymerase II",
  "term_id": "GO:0045944",
  "gene_symbol": "ASCL3"
}